{
  "term_id": "UNKNOWN:0003",
  "gene": "UniProtKB:A0A1B0GW64",
  "gene_name": "Small integral membrane protein 33",
  "gene_symbol": "SMIM33",
  "term_label": "Unknown cellular component"
}